{
  "term_label": "U1 snRNP",
  "term_id": "GO:0005685",
  "gene_name": "Small nuclear ribonucleoprotein G",
  "gene": "UniProtKB:P62308",
  "gene_symbol": "SNRPG"
}